{
  "gene_symbol": "REXO2",
  "term_id": "GO:0005739",
  "gene_name": "Oligoribonuclease, mitochondrial",
  "gene": "UniProtKB:Q9Y3B8",
  "term_label": "mitochondrion"
}